{
  "gene": "UniProtKB:Q6IQ55",
  "gene_name": "Tau-tubulin kinase 2",
  "gene_symbol": "TTBK2",
  "term_label": "cilium assembly",
  "term_id": "GO:0060271"
}